4-chlorobenzoyl-CoA dehalogenase activity [GO:0018787] (molecular function) Relationships: is a type of GO:0019120 Also known as: 4-chlorobenzoyl CoA chlorohydrolase activity Sources: RHEA:14853 Definition: Catalysis of the reaction: 4-chlorobenzoyl-CoA + H2O = 4-hydroxybenzoyl-CoA + chloride + H+.